{
  "term_id": "GO:0016020",
  "term_label": "membrane",
  "gene_name": "Diacylglycerol kinase epsilon",
  "gene": "UniProtKB:P52429",
  "gene_symbol": "DGKE"
}